isopentenyl diphosphate biosynthetic process, methylerythritol 4-phosphate pathway [GO:0019288] (biological process) Relationships: is a type of GO:0009240; is a type of glyceraldehyde-3-phosphate metabolic process [GO:0019682] Regulation: regulated by regulation of isopentenyl diphosphate biosynthetic process, methylerythritol 4-phosphate pathway [GO:0010322]; RO_0002212 by negative regulation of isopentenyl diphosphate biosynthetic process, methylerythritol 4-phosphate pathway [GO:0010323] Definition: The chemical reactions and pathways resulting in the formation of isopentenyl diphosphate by the mevalonate-independent pathway. Isopentenyl diphosphate (IPP) is the fundamental unit in isoprenoid biosynthesis and is biosynthesized from pyruvate and glyceraldehyde 3-phosphate via intermediates, including 1-deoxy-D-xylulose 5-phosphate. Subtypes: GO:0051484 Also known as: isopentenyl diphosphate anabolism, mevalonate-independent pathway, isopentenyl diphosphate biosynthesis, mevalonate-independent, isopentenyl diphosphate biosynthesis, non-mevalonate pathway, isopentenyl diphosphate biosynthetic process via 1-deoxy-D-xylulose 5-phosphate, isopentenyl diphosphate biosynthetic process, MEP pathway, isopentenyl diphosphate biosynthetic process, mevalonate-independent, isopentenyl diphosphate biosynthetic process, mevalonate-independent pathway, isopentenyl diphosphate biosynthetic process, non-mevalonate pathway, isopentenyl diphosphate formation, mevalonate-independent pathway, isopentenyl diphosphate synthesis, mevalonate-independent pathway, mevalonate-independent isopentenyl diphosphate biosynthesis, mevalonate-independent isopentenyl diphosphate biosynthetic process, non-MVA pathway References: PMID:18948055 Sources: GOC:go_curators, MetaCyc:NONMEVIPP-PWY